Fas-activated serine/threonine kinase activity [GO:0033867] (MF) Also known as: ATP:Fas-activated serine/threonine protein phosphotransferase activity, FAST, FASTK, STK10 Relationships: is a type of protein serine/threonine kinase activity [GO:0004674] Definition: Catalysis of the reaction: ATP + Fas-activated serine/threonine protein = ADP + Fas-activated serine/threonine phosphoprotein. Sources: EC:2.7.11.8